positive regulation of clathrin coat assembly [GO:1905445] (biological process) Definition: Any process that activates or increases the frequency, rate or extent of clathrin coat assembly. Relationships: is a type of positive regulation of protein-containing complex assembly [GO:0031334]; is a type of regulation of clathrin coat assembly [GO:1905443]; positively regulates clathrin coat assembly [GO:0048268] Also known as: positive regulation of clathrin cage assembly, up regulation of clathrin cage assembly, up regulation of clathrin coat assembly, up-regulation of clathrin cage assembly, up-regulation of clathrin coat assembly, upregulation of clathrin cage assembly, upregulation of clathrin coat assembly, activation of clathrin cage assembly, activation of clathrin coat assembly References: PMID:15533940 Sources: GOC:PARL, GOC:TermGenie, GOC:bf, GO_REF:0000058